{
  "term_label": "late endosome to vacuole transport via multivesicular body sorting pathway",
  "gene_symbol": "CHMP7",
  "gene_name": "Charged multivesicular body protein 7",
  "gene": "UniProtKB:Q8WUX9",
  "term_id": "GO:0032511"
}